1-phosphatidyl-1D-myo-inositol 4,5-bisphosphate biosynthetic process [GO:1902635] (biological process) Definition: The chemical reactions and pathways resulting in the formation of 1-phosphatidyl-1D-myo-inositol 4,5-bisphosphate. References: PMID:22562153 Sources: GOC:TermGenie, GOC:di, GO_REF:0000068 Also known as: 1-phosphatidyl-1D-myo-inositol 4,5-bisphosphate anabolism, 1-phosphatidyl-1D-myo-inositol 4,5-bisphosphate biosynthesis, 1-phosphatidyl-1D-myo-inositol 4,5-bisphosphate formation, 1-phosphatidyl-1D-myo-inositol 4,5-bisphosphate synthesis, PtdIns(4,5)P(2) biosynthesis, phosphatidylinositol-4,5-bisphosphate biosynthesis Relationships: is a type of phosphatidylinositol phosphate biosynthetic process [GO:0046854]; is a type of 1-phosphatidyl-1D-myo-inositol 4,5-bisphosphate metabolic process [GO:1902633] Regulation: regulated by regulation of 1-phosphatidyl-1D-myo-inositol 4,5-bisphosphate biosynthetic process [GO:1902646]; negatively regulated by negative regulation of 1-phosphatidyl-1D-myo-inositol 4,5-bisphosphate biosynthetic process [GO:1902647]; RO_0002213 by positive regulation of 1-phosphatidyl-1D-myo-inositol 4,5-bisphosphate biosynthetic process [GO:1902648]